p-cymene catabolic process [GO:0019334] (biological process) Definition: The chemical reactions and pathways resulting in the breakdown of p-cymene, 1-methyl-4-isopropylbenzene, one of the alkyl-substituted aromatic hydrocarbons found in volatile oils from over 100 plants. Also known as: p-cymene breakdown, p-cymene catabolism, p-cymene degradation Relationships: is a type of GO:0043694; is a type of toluene-containing compound catabolic process [GO:0072491] Sources: GOC:ai